{
  "gene_symbol": "XYLT2",
  "gene_name": "Xylosyltransferase 2",
  "term_label": "Unknown cellular component",
  "gene": "UniProtKB:Q9H1B5",
  "term_id": "UNKNOWN:0003"
}